axonemal microtubule doublet ribbon [GO:0160115] (cellular component) Definition: The 3 protofilaments A11, A12, and A13 of the A tubule along with associated inner sheath microtuble inner proteins (MIPs), either in the lumen of the A tubule or of the B tubule, which stabilize these three filiments within the axonemal doublet microtubule. The ribbon protofilaments separate the lumens of the A and B tubules. References: PMID:1262413, PMID:29430673 Sources: GOC:krc Relationships: is_a cellular anatomical structure [GO:0110165]; is part of axonemal doublet microtubule [GO:0097545]